error-free postreplication DNA repair [GO:0042275] (biological process) Subtypes: single-strand break repair via homologous recombination [GO:1990396] References: PMID:11459630 Sources: GOC:elh, GOC:jl Note: Note that 'error-free' does not mean that literally zero errors occur during DNA synthesis, but that the error rate is low, comparable to that of DNA synthesis during replication. Definition: The conversion of DNA-damage induced single-stranded gaps into large molecular weight DNA via processes such as template switching, which does not remove the replication-blocking lesions but does not increase the endogenous mutation rate. Relationships: is_a DNA damage tolerance [GO:0006301] Also known as: error-free PRR, error-free replication restart